5-methylthiopropyl glucosinolate S-oxygenase activity [GO:0080104] (molecular function) Relationships: is a type of GO:0016705 References: PMID:18799661 Definition: Catalysis of the reaction: 5-methylthiopropyl-glucosinolate = 5-methylsulfinylpropyl-glucosinolate.